{
  "gene_name": "Thiol S-methyltransferase TMT1B",
  "term_label": "Unknown cellular component",
  "gene": "UniProtKB:Q6UX53",
  "gene_symbol": "TMT1B",
  "term_id": "UNKNOWN:0003"
}